spinal cord motor neuron cell fate specification [GO:0021520] (BP) Relationships: is a type of neuron fate specification [GO:0048665]; is part of spinal cord motor neuron differentiation [GO:0021522] Definition: The process in which a cell becomes capable of differentiating autonomously into a motor neuron in an environment that is neutral with respect to the developmental pathway. Sources: GOC:cls, GOC:dgh, GOC:dph, GOC:jid, GO_REF:0000021